{
  "term_id": "GO:0006355",
  "gene_name": "Zinc finger and BTB domain-containing protein 38",
  "term_label": "regulation of DNA-templated transcription",
  "gene_symbol": "ZBTB38",
  "gene": "UniProtKB:Q8NAP3"
}